{
  "term_id": "GO:0007155",
  "gene": "UniProtKB:Q15582",
  "gene_name": "Transforming growth factor-beta-induced protein ig-h3",
  "gene_symbol": "TGFBI",
  "term_label": "cell adhesion"
}